{
  "gene_name": "DNA damage-inducible transcript 3 protein",
  "gene_symbol": "DDIT3",
  "gene": "UniProtKB:P35638",
  "term_label": "intrinsic apoptotic signaling pathway in response to endoplasmic reticulum stress",
  "term_id": "GO:0070059"
}